RNA sequestering activity [GO:0140610] (MF) Relationships: is a type of GO:0140313; has part RNA binding [GO:0003723] References: PMID:23334420, PMID:29084823 Definition: Binding to a specific RNA molecule to prevent it from interacting with other partners or to inhibit its localization to the area of the cell or complex where it is active.